{
  "term_id": "UNKNOWN:0001",
  "gene": "UniProtKB:O75431",
  "gene_name": "Metaxin-2",
  "term_label": "Unknown molecular function",
  "gene_symbol": "MTX2"
}